Golgi medial cisterna-derived vesicle fusion with Golgi cis cisterna membrane [GO:1990690] (biological process) Also known as: Golgi apparatus medial cisterna-derived vesicle fusion with Golgi apparatus cis cisterna membrane, medial-Golgi cisterna-derived vesicle fusion with cis-Golgi cisterna membrane Relationships: is a type of GO:0048210; is a type of vesicle fusion with Golgi apparatus [GO:0048280]; is part of retrograde transport, vesicle recycling within Golgi [GO:0000301] References: PMID:16038056, PMID:24119662 Sources: GOC:bhm Definition: The joining of the lipid bilayer membrane around a Golgi medial cisterna-derived vesicle to the lipid bilayer membrane around the Golgi cis cisterna. Such vesicles include COPI-coated transport vesicles involved in retrograde transport.